{
  "gene_name": "Reversion-inducing cysteine-rich protein with Kazal motifs",
  "term_label": "endopeptidase inhibitor activity",
  "term_id": "GO:0004866",
  "gene": "UniProtKB:O95980",
  "gene_symbol": "RECK"
}